{
  "term_label": "positive regulation of MAPK cascade",
  "gene_name": "Proto-oncogene serine_threonine-protein kinase mos",
  "term_id": "GO:0043410",
  "gene_symbol": "MOS",
  "gene": "UniProtKB:P00540"
}